{
  "term_id": "UNKNOWN:0002",
  "gene_symbol": "SSX9P",
  "term_label": "Unknown biological process",
  "gene_name": "Putative protein SSX9",
  "gene": "UniProtKB:Q7RTT3"
}